{
  "term_id": "GO:0051726",
  "term_label": "regulation of cell cycle",
  "gene_symbol": "COPS5",
  "gene": "UniProtKB:Q92905",
  "gene_name": "COP9 signalosome complex subunit 5"
}